regulation of protein adenylylation [GO:1900722] (biological process) Definition: Any process that modulates the frequency, rate or extent of protein adenylylation. Sources: GOC:TermGenie Relationships: is a type of regulation of protein modification process [GO:0031399]; regulates protein adenylylation [GO:0018117] Also known as: regulation of protein AMPylation, regulation of protein adenylation, regulation of protein amino acid adenylylation Subtypes: negative regulation of protein adenylylation [GO:1900723], positive regulation of protein adenylylation [GO:1900724]